{
  "gene_name": "Protein phosphatase 1 regulatory subunit 7",
  "gene_symbol": "PPP1R7",
  "term_id": "GO:0005737",
  "gene": "UniProtKB:Q15435",
  "term_label": "cytoplasm"
}